{
  "term_label": "Unknown cellular component",
  "gene": "UniProtKB:Q9Y450",
  "term_id": "UNKNOWN:0003",
  "gene_name": "HBS1-like protein",
  "gene_symbol": "HBS1L"
}